{
  "term_id": "GO:0005737",
  "gene_symbol": "AFMID",
  "term_label": "cytoplasm",
  "gene_name": "Kynurenine formamidase",
  "gene": "UniProtKB:Q63HM1"
}